{
  "term_id": "GO:0005829",
  "gene": "UniProtKB:Q96CS2",
  "term_label": "cytosol",
  "gene_name": "HAUS augmin-like complex subunit 1",
  "gene_symbol": "HAUS1"
}